{
  "gene_symbol": "CNGA2",
  "term_label": "monoatomic cation transmembrane transport",
  "term_id": "GO:0098655",
  "gene": "UniProtKB:Q16280",
  "gene_name": "Cyclic nucleotide-gated olfactory channel"
}